peptidyl-lysine deacetylation [GO:0034983] (biological process) Relationships: is a type of GO:0006476; is a type of peptidyl-lysine modification [GO:0018205] Also known as: protein lysine acetylation Sources: GOC:BHF, GOC:mah Definition: The removal of an acetyl group from an acetylated lysine residue in a peptide or protein.